negative regulation of convergent extension involved in somitogenesis [GO:1904128] (biological process) Definition: Any process that stops, prevents or reduces the frequency, rate or extent of convergent extension involved in somitogenesis. References: PMID:24892953 Sources: GOC:TermGenie, GOC:dph, GO_REF:0000058 Also known as: down regulation of convergent extension involved in somitogenesis, down-regulation of convergent extension involved in somitogenesis, downregulation of convergent extension involved in somitogenesis, inhibition of convergent extension involved in somitogenesis Relationships: is a type of negative regulation of convergent extension involved in axis elongation [GO:1901233]; is a type of GO:1904104; is a type of GO:1904127; negatively regulates convergent extension involved in somitogenesis [GO:0090246]